sebum secreting cell proliferation [GO:1990654] (biological process) Regulation: regulated by regulation of sebum secreting cell proliferation [GO:1904002]; negatively regulated by negative regulation of sebum secreting cell proliferation [GO:1904003]; positively regulated by positive regulation of sebum secreting cell proliferation [GO:1904004] References: PMID:16901790, PMID:18474083 Sources: GOC:hjd Also known as: sebocyte proliferation Definition: The multiplication or reproduction of sebocytes by cell division, resulting in the expansion of their population. A sebocyte is an epithelial cell that makes up the sebaceous glands, and secrete sebum. Relationships: is a type of GO:0050673